myeloid dendritic cell cytokine production [GO:0002372] (biological process) Relationships: is a type of GO:0002371; is a type of GO:0002444; is a type of myeloid leukocyte cytokine production [GO:0061082] Definition: Any process that contributes to cytokine production by a myeloid dendritic cell. Regulation: regulated by regulation of myeloid dendritic cell cytokine production [GO:0002733]; RO_0002212 by negative regulation of myeloid dendritic cell cytokine production [GO:0002734]; positively regulated by positive regulation of myeloid dendritic cell cytokine production [GO:0002735] Note: Note that this term is in the subset of terms that should not be used for direct gene product annotation. Instead, select one of the 'regulation' children terms. Sources: GOC:add, ISBN:0781735149